{
  "term_label": "Unknown molecular function",
  "gene_name": "G antigen 12I",
  "gene": "UniProtKB:P0CL82",
  "gene_symbol": "GAGE12I",
  "term_id": "UNKNOWN:0001"
}